{
  "term_label": "Unknown biological process",
  "term_id": "UNKNOWN:0002",
  "gene_name": "Protein TNT",
  "gene_symbol": "C16orf82",
  "gene": "UniProtKB:Q7Z2V1"
}